{
  "gene_name": "E3 ubiquitin-protein ligase ARIH1",
  "gene": "UniProtKB:Q9Y4X5",
  "term_id": "GO:0006511",
  "gene_symbol": "ARIH1",
  "term_label": "ubiquitin-dependent protein catabolic process"
}